{
  "gene_name": "Pericentrin",
  "term_label": "microtubule nucleation",
  "gene_symbol": "PCNT",
  "gene": "UniProtKB:O95613",
  "term_id": "GO:0007020"
}